{
  "term_label": "endocytic vesicle",
  "gene": "UniProtKB:Q9H4M9",
  "gene_symbol": "EHD1",
  "term_id": "GO:0030139",
  "gene_name": "EH domain-containing protein 1"
}